{
  "gene_symbol": "FFAR4",
  "gene_name": "Free fatty acid receptor 4",
  "gene": "UniProtKB:Q5NUL3",
  "term_label": "plasma membrane",
  "term_id": "GO:0005886"
}